division septum site selection [GO:0000918] (BP) Definition: The process of marking the site where a division septum will form. Also known as: septin assembly and septum biosynthesis, septin assembly and septum formation, selection of site for barrier cell septum biosynthesis, selection of site for barrier cell septum formation, selection of site for division septum formation, septum positioning Relationships: is a type of GO:0032506; is part of division septum assembly [GO:0000917] Sources: GOC:clt